{
  "gene_symbol": "SRSF3",
  "term_id": "GO:0000381",
  "gene": "UniProtKB:P84103",
  "term_label": "regulation of alternative mRNA splicing, via spliceosome",
  "gene_name": "Serine_arginine-rich splicing factor 3"
}